3-oxoadipate enol-lactonase activity [GO:0047570] (molecular function) Relationships: is a type of carboxylic ester hydrolase activity [GO:0052689] Definition: Catalysis of the reaction: 3-oxoadipate enol-lactone + H2O = 3-oxoadipate. Also known as: 3-ketoadipate enol-lactonase activity, 3-oxoadipic enol-lactone hydrolase activity, 4-carboxymethylbut-3-en-4-olide enol-lactonohydrolase activity, beta-ketoadipate enol-lactone hydrolase activity, beta-ketoadipic enol-lactone hydrolase activity, carboxymethylbutenolide lactonase activity Sources: EC:3.1.1.24, MetaCyc:3-OXOADIPATE-ENOL-LACTONASE-RXN